metal ion binding [GO:0046872] (molecular function) Relationships: is a type of GO:0043169 Subtypes: magnesium ion binding [GO:0000287], calcium ion binding [GO:0005509], alkali metal ion binding [GO:0031420], lead ion binding [GO:0032791], metal chelating activity [GO:0046911], transition metal ion binding [GO:0046914] Also known as: metal binding, heavy metal binding Sources: GOC:ai Definition: Binding to a metal ion.